{
  "term_label": "endoplasmic reticulum",
  "gene_name": "DnaJ homolog subfamily B member 9",
  "term_id": "GO:0005783",
  "gene": "UniProtKB:Q9UBS3",
  "gene_symbol": "DNAJB9"
}